positive regulation of protein homooligomerization [GO:0032464] (biological process) Definition: Any process that activates or increases the frequency, rate or extent of protein homooligomerization. Sources: GOC:mah Subtypes: GO:1901095 Relationships: is a type of GO:0032461; is a type of regulation of protein homooligomerization [GO:0032462]; positively regulates GO:0051260 Also known as: up regulation of protein homooligomerization, up-regulation of protein homooligomerization, upregulation of protein homooligomerization, activation of protein homooligomerization, stimulation of protein homooligomerization, induction of protein homooligomerization